{
  "gene_name": "Claudin-10",
  "gene": "UniProtKB:P78369",
  "gene_symbol": "CLDN10",
  "term_label": "paracellular transport",
  "term_id": "GO:0160184"
}